{
  "gene_symbol": "TM6SF2",
  "term_id": "GO:0019216",
  "gene": "UniProtKB:Q9BZW4",
  "term_label": "regulation of lipid metabolic process",
  "gene_name": "Transmembrane 6 superfamily member 2"
}